{
  "gene_symbol": "FER1L6-AS1",
  "term_id": "UNKNOWN:0002",
  "term_label": "Unknown biological process",
  "gene": "UniProtKB:Q8NA97",
  "gene_name": "Putative uncharacterized protein FER1L6-AS1"
}